{
  "term_label": "nucleus",
  "gene_name": "Protein C-ets-1",
  "term_id": "GO:0005634",
  "gene": "UniProtKB:P14921",
  "gene_symbol": "ETS1"
}